{
  "gene_name": "Myocyte-specific enhancer factor 2D",
  "term_id": "GO:0045944",
  "gene_symbol": "MEF2D",
  "term_label": "positive regulation of transcription by RNA polymerase II",
  "gene": "UniProtKB:Q14814"
}